{
  "gene_name": "Testis-specific basic protein Y 1",
  "term_label": "brain development",
  "gene": "UniProtKB:O14598",
  "term_id": "GO:0007420",
  "gene_symbol": "VCY"
}